{
  "gene_symbol": "SBF2",
  "term_label": "membrane",
  "term_id": "GO:0016020",
  "gene_name": "Myotubularin-related protein 13",
  "gene": "UniProtKB:Q86WG5"
}